{
  "term_label": "lipopolysaccharide receptor complex",
  "term_id": "GO:0046696",
  "gene_name": "Toll-like receptor 4",
  "gene_symbol": "TLR4",
  "gene": "UniProtKB:O00206"
}